{
  "term_id": "UNKNOWN:0001",
  "gene_name": "Uncharacterized protein UMODL1-AS1",
  "gene": "UniProtKB:Q8N2C9",
  "term_label": "Unknown molecular function",
  "gene_symbol": "UMODL1-AS1"
}